riboflavin transmembrane transporter activity [GO:0032217] (molecular function) Relationships: is a type of vitamin transmembrane transporter activity [GO:0090482]; is part of riboflavin transport [GO:0032218] Definition: Enables the transfer of riboflavin from one side of a membrane to the other. Riboflavin (vitamin B2) is a water-soluble B-complex vitamin, converted in the cell to FMN and FAD, cofactors required for the function of flavoproteins. References: PMID:16204239 Sources: GOC:rn Also known as: riboflavin transporter activity